{
  "gene_symbol": "DACH1",
  "term_label": "transcription regulator complex",
  "gene_name": "Dachshund homolog 1",
  "gene": "UniProtKB:Q9UI36",
  "term_id": "GO:0005667"
}